{
  "term_id": "GO:0005634",
  "term_label": "nucleus",
  "gene": "UniProtKB:Q8TBC4",
  "gene_symbol": "UBA3",
  "gene_name": "NEDD8-activating enzyme E1 catalytic subunit"
}